{
  "gene_name": "Putative homeobox protein NANOG2",
  "term_id": "GO:0000981",
  "term_label": "DNA-binding transcription factor activity, RNA polymerase II-specific",
  "gene_symbol": "NANOGP1",
  "gene": "UniProtKB:Q8N7R0"
}